{
  "gene": "UniProtKB:P0DTA3",
  "term_id": "UNKNOWN:0002",
  "gene_symbol": "SPDYE11",
  "gene_name": "Putative speedy protein E11",
  "term_label": "Unknown biological process"
}